{
  "gene_name": "Myristoylated alanine-rich C-kinase substrate",
  "term_id": "GO:0032432",
  "gene_symbol": "MARCKS",
  "gene": "UniProtKB:P29966",
  "term_label": "actin filament bundle"
}